activin receptor signaling pathway [GO:0032924] (biological process) Regulation: regulated by regulation of activin receptor signaling pathway [GO:0032925]; negatively regulated by negative regulation of activin receptor signaling pathway [GO:0032926]; positively regulated by positive regulation of activin receptor signaling pathway [GO:0032927] Definition: The series of molecular signals initiated by an extracellular ligand binding to an activin receptor on the surface of a target cell, and ending with the regulation of a downstream cellular process, e.g. transcription. Also known as: activin receptor signalling pathway Relationships: is a type of transforming growth factor beta receptor superfamily signaling pathway [GO:0141091] Subtypes: nodal signaling pathway [GO:0038092] Sources: GOC:rl, GOC:signaling